{
  "term_label": "prostaglandin biosynthetic process",
  "gene": "UniProtKB:Q15185",
  "gene_symbol": "PTGES3",
  "term_id": "GO:0001516",
  "gene_name": "Prostaglandin E synthase 3"
}